{
  "term_label": "ubiquitin ligase complex scaffold activity",
  "gene_symbol": "CUL4B",
  "gene_name": "Cullin-4B",
  "term_id": "GO:0160072",
  "gene": "UniProtKB:Q13620"
}